positive regulation of olefin biosynthetic process [GO:1900913] (biological process) Relationships: is a type of positive regulation of biosynthetic process [GO:0009891]; is a type of regulation of olefin biosynthetic process [GO:1900911]; positively regulates olefin biosynthetic process [GO:1900674] Also known as: up regulation of olefin biosynthetic process, up-regulation of olefin biosynthetic process, upregulation of olefin biosynthetic process, activation of olefin anabolism, activation of olefin biosynthesis, activation of olefin biosynthetic process, activation of olefin formation, activation of olefin synthesis, positive regulation of olefin anabolism, positive regulation of olefin biosynthesis, positive regulation of olefin formation, positive regulation of olefin synthesis, up regulation of olefin anabolism, up regulation of olefin biosynthesis, up regulation of olefin formation, up regulation of olefin synthesis, up-regulation of olefin anabolism, up-regulation of olefin biosynthesis, up-regulation of olefin formation, up-regulation of olefin synthesis, upregulation of olefin anabolism, upregulation of olefin biosynthesis, upregulation of olefin formation, upregulation of olefin synthesis Sources: GOC:TermGenie, GOC:mengo_curators Definition: Any process that activates or increases the frequency, rate or extent of olefin biosynthetic process. Subtypes: positive regulation of ethylene biosynthetic process [GO:0010365], positive regulation of octadecene biosynthetic process [GO:1900916], positive regulation of nonadec-1-ene biosynthetic process [GO:1900937], GO:1900943, GO:1900949, positive regulation of 18-methylnonadec-1-ene biosynthetic process [GO:1900952], GO:1900958